Kv4.2-KChIP2 channel complex [GO:0071193] (cellular component) References: PMID:15356203 Relationships: is a type of voltage-gated potassium channel complex [GO:0008076] Definition: A voltage-gated potassium channel complex that contains the Kv channel interacting protein KChIP2 associated with the channel via interaction with the Kv alpha subunit 4.2.